osmoregulated periplasmic glucan catabolic process [GO:1900726] (biological process) Relationships: is a type of glucan catabolic process [GO:0009251] Sources: GOC:TermGenie, GOC:yaf Also known as: osmoregulated periplasmic glucan breakdown, osmoregulated periplasmic glucan catabolism, osmoregulated periplasmic glucan degradation Definition: The chemical reactions and pathways resulting in the breakdown of osmoregulated periplasmic glucan.